negative regulation of dendritic cell dendrite assembly [GO:2000548] (biological process) Definition: Any process that stops, prevents or reduces the frequency, rate or extent of dendritic cell dendrite assembly. Sources: GOC:obol Also known as: negative regulation of dendritic extension Relationships: is_a GO:0120033; is a type of regulation of dendritic cell dendrite assembly [GO:2000547]; negatively regulates dendritic cell dendrite assembly [GO:0097026]